{
  "gene_name": "Zinc finger protein 296",
  "term_label": "negative regulation of dendrite development",
  "term_id": "GO:2000171",
  "gene_symbol": "ZNF296",
  "gene": "UniProtKB:Q8WUU4"
}